{
  "gene_name": "Prelamin-A_C",
  "term_label": "nuclear pore localization",
  "term_id": "GO:0051664",
  "gene_symbol": "LMNA",
  "gene": "UniProtKB:P02545"
}